{
  "gene_symbol": "SLC7A2",
  "term_id": "GO:0015189",
  "gene": "UniProtKB:P52569",
  "gene_name": "Cationic amino acid transporter 2",
  "term_label": "L-lysine transmembrane transporter activity"
}